{
  "term_label": "homologous chromosome segregation",
  "term_id": "GO:0045143",
  "gene_symbol": "PTTG3P",
  "gene": "UniProtKB:Q9NZH4",
  "gene_name": "Putative pituitary tumor-transforming gene 3 protein"
}